{
  "gene_name": "EH domain-containing protein 3",
  "term_label": "protein-macromolecule adaptor activity",
  "term_id": "GO:0030674",
  "gene_symbol": "EHD3",
  "gene": "UniProtKB:Q9NZN3"
}